{
  "term_label": "Unknown biological process",
  "gene_name": "Keratin-associated protein 22-2",
  "gene": "UniProtKB:Q3LI68",
  "gene_symbol": "KRTAP22-2",
  "term_id": "UNKNOWN:0002"
}